{
  "term_id": "GO:0097422",
  "term_label": "tubular endosome",
  "gene_symbol": "ANKRD27",
  "gene": "UniProtKB:Q96NW4",
  "gene_name": "Ankyrin repeat domain-containing protein 27"
}